all-trans-retinol dehydrogenase (NAD+) activity [GO:0004745] (molecular function) Also known as: all-trans retinol dehydrogenase activity, retinal reductase activity, retinene reductase activity, retinol (vitamin A1) dehydrogenase activity, retinol dehydrogenase activity Definition: Catalysis of the reaction: all-trans-retinol--[retinol-binding protein] + NAD+ = all-trans-retinal--[retinol-binding protein] + H+ + NADH. Recognizes the substrate both in free form and when bound to cellular-retinol-binding-protein (CRBP1), but has higher affinity for the bound form. Relationships: is a type of alcohol dehydrogenase (NAD+) activity [GO:0004022] Sources: RHEA:48488